{
  "gene_symbol": "PSMD14",
  "gene": "UniProtKB:O00487",
  "term_id": "GO:0008541",
  "term_label": "proteasome regulatory particle, lid subcomplex",
  "gene_name": "26S proteasome non-ATPase regulatory subunit 14"
}